{
  "term_id": "GO:0000086",
  "gene_name": "Serine_threonine-protein kinase BRSK1",
  "gene": "UniProtKB:Q8TDC3",
  "term_label": "G2/M transition of mitotic cell cycle",
  "gene_symbol": "BRSK1"
}